{
  "term_label": "P-type divalent copper transporter activity",
  "gene_name": "Copper-transporting ATPase 1",
  "gene": "UniProtKB:Q04656",
  "term_id": "GO:0043682",
  "gene_symbol": "ATP7A"
}